{
  "term_label": "nucleus",
  "gene_symbol": "CIART",
  "gene": "UniProtKB:Q8N365",
  "term_id": "GO:0005634",
  "gene_name": "Circadian-associated transcriptional repressor"
}